{
  "gene": "UniProtKB:P0C7M7",
  "term_id": "GO:0006633",
  "term_label": "fatty acid biosynthetic process",
  "gene_symbol": "ACSM4",
  "gene_name": "Acyl-coenzyme A synthetase ACSM4, mitochondrial"
}